{
  "gene": "UniProtKB:P54274",
  "term_label": "nuclear telomere cap complex",
  "term_id": "GO:0000783",
  "gene_name": "Telomeric repeat-binding factor 1",
  "gene_symbol": "TERF1"
}